{
  "gene": "UniProtKB:A0A075B6N4",
  "term_label": "Unknown molecular function",
  "term_id": "UNKNOWN:0001",
  "gene_name": "T cell receptor beta variable 25-1",
  "gene_symbol": "TRBV25-1"
}